{
  "term_label": "cytoplasm",
  "gene_name": "Rho GTPase-activating protein 18",
  "gene": "UniProtKB:Q8N392",
  "gene_symbol": "ARHGAP18",
  "term_id": "GO:0005737"
}